{
  "gene": "UniProtKB:Q15620",
  "term_label": "Unknown cellular component",
  "term_id": "UNKNOWN:0003",
  "gene_symbol": "OR8B8",
  "gene_name": "Olfactory receptor 8B8"
}